{
  "gene": "UniProtKB:Q9H2K0",
  "term_id": "GO:0032790",
  "term_label": "ribosome disassembly",
  "gene_name": "Translation initiation factor IF-3, mitochondrial",
  "gene_symbol": "MTIF3"
}